pyrimidine ribonucleotide biosynthetic process [GO:0009220] (biological process) Also known as: pyrimidine ribonucleotide anabolism, pyrimidine ribonucleotide biosynthesis, pyrimidine ribonucleotide formation, pyrimidine ribonucleotide synthesis Relationships: is a type of pyrimidine nucleotide biosynthetic process [GO:0006221]; is a type of pyrimidine ribonucleotide metabolic process [GO:0009218]; is a type of GO:0009260 Sources: GOC:go_curators, ISBN:0198506732 Definition: The chemical reactions and pathways resulting in the formation of a pyrimidine ribonucleotide, a compound consisting of nucleoside (a pyrimidine base linked to a ribose sugar) esterified with a phosphate group at either the 3' or 5'-hydroxyl group of the sugar. Subtypes: UMP biosynthetic process [GO:0006222], UDP biosynthetic process [GO:0006225], UTP biosynthetic process [GO:0006228], GO:0006230, GO:0006232, GO:0006234, CTP biosynthetic process [GO:0006241], CMP biosynthetic process [GO:0009224], pyrimidine ribonucleotide salvage [GO:0010138], GO:0046705